{
  "gene": "UniProtKB:Q96BD8",
  "gene_symbol": "SKA1",
  "term_id": "GO:0008017",
  "gene_name": "Spindle and kinetochore-associated protein 1",
  "term_label": "microtubule binding"
}